{
  "gene_symbol": "IL3RA",
  "term_id": "GO:0004896",
  "gene": "UniProtKB:P26951",
  "term_label": "cytokine receptor activity",
  "gene_name": "Interleukin-3 receptor subunit alpha"
}